{
  "gene_name": "Rhox homeobox family member 1 pseudogene 3",
  "term_label": "Unknown molecular function",
  "gene_symbol": "RHOXF1P3",
  "term_id": "UNKNOWN:0001",
  "gene": "UniProtKB:A0A994J3T1"
}